{
  "gene_symbol": "PTPN2",
  "term_label": "negative regulation of ERK1 and ERK2 cascade",
  "term_id": "GO:0070373",
  "gene_name": "Tyrosine-protein phosphatase non-receptor type 2",
  "gene": "UniProtKB:P17706"
}